{
  "gene_name": "Cytochrome P450 2C19",
  "term_id": "GO:0019373",
  "gene_symbol": "CYP2C19",
  "gene": "UniProtKB:P33261",
  "term_label": "epoxygenase P450 pathway"
}